{
  "term_label": "plasma membrane",
  "gene": "UniProtKB:O14917",
  "gene_name": "Protocadherin-17",
  "term_id": "GO:0005886",
  "gene_symbol": "PCDH17"
}